{
  "gene_symbol": "CHIC2",
  "term_label": "Unknown molecular function",
  "gene": "UniProtKB:Q9UKJ5",
  "term_id": "UNKNOWN:0001",
  "gene_name": "Cysteine-rich hydrophobic domain-containing protein 2"
}